{
  "term_id": "GO:0006382",
  "term_label": "adenosine to inosine editing",
  "gene": "UniProtKB:Q96M93",
  "gene_symbol": "ADAD1",
  "gene_name": "Adenosine deaminase domain-containing protein 1"
}